{
  "gene": "UniProtKB:A0A1W2PPK0",
  "gene_symbol": "CPHXL2",
  "gene_name": "Cytoplasmic polyadenylated homeobox-like protein 2",
  "term_label": "regulation of transcription by RNA polymerase II",
  "term_id": "GO:0006357"
}